{
  "term_label": "type I interferon receptor binding",
  "gene_symbol": "IFNE",
  "gene": "UniProtKB:Q86WN2",
  "term_id": "GO:0005132",
  "gene_name": "Interferon epsilon"
}